{
  "gene_name": "NACHT, LRR and PYD domains-containing protein 8",
  "term_id": "GO:0005737",
  "term_label": "cytoplasm",
  "gene_symbol": "NLRP8",
  "gene": "UniProtKB:Q86W28"
}